{
  "gene": "UniProtKB:O60343",
  "term_id": "GO:0005794",
  "gene_symbol": "TBC1D4",
  "term_label": "Golgi apparatus",
  "gene_name": "TBC1 domain family member 4"
}